positive regulation of activated T cell autonomous cell death [GO:0070241] (biological process) Definition: Any process that activates or increases the frequency, rate or extent of activated T cell autonomous cell death. Sources: GOC:add, GOC:mtg_apoptosis, ISBN:0781765196 Also known as: positive regulation of ACAD, positive regulation of activated T cell apoptosis, positive regulation of activated cell autonomous cell death, positive regulation of activated T lymphocyte autonomous cell death, positive regulation of activated T-cell autonomous cell death, positive regulation of activated T-lymphocyte autonomous cell death, up regulation of activated T cell autonomous cell death, up-regulation of activated T cell autonomous cell death, upregulation of activated T cell autonomous cell death, activation of activated T cell autonomous cell death, stimulation of activated T cell autonomous cell death Relationships: is a type of positive regulation of immune system process [GO:0002684]; is a type of positive regulation of T cell apoptotic process [GO:0070234]; is a type of GO:0070239; positively regulates activated T cell autonomous cell death [GO:0070238]